{
  "gene_name": "Protein NLRC5",
  "gene_symbol": "NLRC5",
  "term_label": "Unknown molecular function",
  "term_id": "UNKNOWN:0001",
  "gene": "UniProtKB:Q86WI3"
}